embryonic foregut morphogenesis [GO:0048617] (biological process) Sources: GOC:jid, GOC:rc Definition: The process in which the anatomical structures of the foregut are generated and organized, during the embryonic phase. Relationships: is a type of embryonic morphogenesis [GO:0048598]; is part of foregut morphogenesis [GO:0007440]